{
  "gene_symbol": "KRT71",
  "term_id": "GO:0031424",
  "gene_name": "Keratin, type II cytoskeletal 71",
  "gene": "UniProtKB:Q3SY84",
  "term_label": "keratinization"
}